{
  "gene": "UniProtKB:A6NGU7",
  "gene_symbol": "LINC01546",
  "term_label": "Unknown biological process",
  "gene_name": "Putative uncharacterized protein encoded by LINC01546",
  "term_id": "UNKNOWN:0002"
}